{
  "gene_symbol": "PM20D1",
  "gene_name": "N-fatty-acyl-amino acid synthase_hydrolase PM20D1",
  "term_id": "GO:0006629",
  "gene": "UniProtKB:Q6GTS8",
  "term_label": "lipid metabolic process"
}